uterine wall growth [GO:0042702] (biological process) Definition: The regrowth of the endometrium and blood vessels in the uterus following menstruation, resulting from a rise in progesterone levels. Sources: GOC:jl Relationships: is a type of ovulation cycle process [GO:0022602]; is a type of developmental growth [GO:0048589]; is part of luteinization [GO:0001553]